{
  "term_label": "adenylate cyclase activity",
  "gene_symbol": "ADCY5",
  "gene": "UniProtKB:O95622",
  "term_id": "GO:0004016",
  "gene_name": "Adenylate cyclase type 5"
}